{
  "gene_symbol": "MT1HL1",
  "gene_name": "Metallothionein 1H-like protein 1",
  "term_label": "cellular response to cadmium ion",
  "term_id": "GO:0071276",
  "gene": "UniProtKB:P0DM35"
}